3'-5' RNA helicase activity [GO:0034458] (molecular function) Sources: GOC:jp Also known as: 3' to 5' RNA helicase activity, ATP-dependent 3' to 5' RNA helicase activity, ATP-dependent 3'-5' RNA helicase activity Relationships: is a type of RNA helicase activity [GO:0003724] Definition: Unwinding of an RNA helix in the 3' to 5' direction, driven by ATP hydrolysis.